{
  "gene_name": "A-kinase anchor protein 8",
  "term_label": "protein kinase A regulatory subunit binding",
  "term_id": "GO:0034237",
  "gene": "UniProtKB:O43823",
  "gene_symbol": "AKAP8"
}